{
  "gene_symbol": "UMODL1-AS1",
  "gene_name": "Uncharacterized protein UMODL1-AS1",
  "gene": "UniProtKB:Q8N2C9",
  "term_label": "Unknown cellular component",
  "term_id": "UNKNOWN:0003"
}